{
  "gene_name": "EEF1A lysine methyltransferase 1",
  "gene": "UniProtKB:Q8WVE0",
  "gene_symbol": "EEF1AKMT1",
  "term_id": "UNKNOWN:0003",
  "term_label": "Unknown cellular component"
}